{
  "term_label": "Unknown cellular component",
  "term_id": "UNKNOWN:0003",
  "gene": "UniProtKB:A6NCN8",
  "gene_name": "Testis-expressed protein 52",
  "gene_symbol": "TEX52"
}